meiotic metaphase II [GO:0007137] (BP) Definition: The cell cycle phase, following prophase II, during which chromosomes become aligned on the equatorial plate of the cell as part of meiosis II. Note: Note that this term should not be used for direct annotation. If you are trying to make an annotation to x phase, it is likely that the correct annotation is 'regulation of x/y phase transition' or to a process which occurs during the reported phase (i.e mitotic DNA replication for mitotic S-phase). To capture the phase when a specific location or process is observed, the phase term can be used in an annotation extension (PMID:24885854) applied to a cellular component term (with the relation exists_during) or a biological process term (with the relation happens_during). Sources: GOC:mtg_cell_cycle Relationships: is a type of metaphase [GO:0051323]; is a type of meiosis II cell cycle phase [GO:0098765]; is part of GO:0051327